{
  "gene": "UniProtKB:Q9Y2C4",
  "gene_symbol": "EXOG",
  "gene_name": "Nuclease EXOG, mitochondrial",
  "term_id": "GO:0005634",
  "term_label": "nucleus"
}